{
  "term_label": "monoamine oxidase activity",
  "gene_symbol": "MAOA",
  "gene_name": "Amine oxidase [flavin-containing] A",
  "gene": "UniProtKB:P21397",
  "term_id": "GO:0097621"
}